{
  "term_label": "Unknown molecular function",
  "term_id": "UNKNOWN:0001",
  "gene": "UniProtKB:Q9UPN9",
  "gene_name": "E3 ubiquitin-protein ligase TRIM33",
  "gene_symbol": "TRIM33"
}